{
  "gene": "UniProtKB:Q96LJ7",
  "gene_symbol": "DHRS1",
  "term_id": "UNKNOWN:0002",
  "gene_name": "Dehydrogenase_reductase SDR family member 1",
  "term_label": "Unknown biological process"
}